{
  "gene": "UniProtKB:O43913",
  "term_id": "GO:0005664",
  "gene_symbol": "ORC5",
  "term_label": "nuclear origin of replication recognition complex",
  "gene_name": "Origin recognition complex subunit 5"
}